{
  "gene_symbol": "PARP1",
  "term_id": "GO:0005730",
  "gene": "UniProtKB:P09874",
  "term_label": "nucleolus",
  "gene_name": "Poly [ADP-ribose] polymerase 1"
}